{
  "gene_symbol": "BSG",
  "term_label": "axon",
  "term_id": "GO:0030424",
  "gene": "UniProtKB:P35613",
  "gene_name": "Basigin"
}